{
  "term_label": "Unknown cellular component",
  "gene_name": "Putative heat shock protein HSP 90-alpha A5",
  "gene_symbol": "HSP90AA5P",
  "term_id": "UNKNOWN:0003",
  "gene": "UniProtKB:Q58FG0"
}